{
  "gene_name": "Dimethyladenosine transferase 2, mitochondrial",
  "term_label": "rRNA (adenine-N6,N6-)-dimethyltransferase activity",
  "gene": "UniProtKB:Q9H5Q4",
  "term_id": "GO:0000179",
  "gene_symbol": "TFB2M"
}